{
  "term_id": "GO:0031119",
  "gene": "UniProtKB:Q9Y606",
  "term_label": "tRNA pseudouridine synthesis",
  "gene_name": "Pseudouridylate synthase 1 homolog",
  "gene_symbol": "PUS1"
}